{
  "gene_symbol": "RNFT1",
  "gene": "UniProtKB:Q5M7Z0",
  "term_id": "GO:0061630",
  "term_label": "ubiquitin protein ligase activity",
  "gene_name": "E3 ubiquitin-protein ligase RNFT1"
}